{
  "gene": "UniProtKB:P49674",
  "term_label": "endocytosis",
  "gene_name": "Casein kinase I isoform epsilon",
  "gene_symbol": "CSNK1E",
  "term_id": "GO:0006897"
}